{
  "gene": "UniProtKB:Q9NPB6",
  "gene_symbol": "PARD6A",
  "term_id": "GO:0005634",
  "term_label": "nucleus",
  "gene_name": "Partitioning defective 6 homolog alpha"
}